head kidney development [GO:0072113] (biological process) Sources: GOC:mtg_kidney_jan10, ZFA:0000669 Definition: The process whose specific outcome is the progression of the head kidney over time, from its formation to the mature structure. The head kidney is a pronephros that consists of fused bilateral lobes located in the anterior part of the kidney. It is analogous to the mammalian bone marrow and the primary site of definitive hematopoiesis. Relationships: is_a hematopoietic or lymphoid organ development [GO:0048534]; is a type of GO:0048793